{
  "term_label": "intracellular protein transport",
  "gene_symbol": "RAB21",
  "gene_name": "Ras-related protein Rab-21",
  "gene": "UniProtKB:Q9UL25",
  "term_id": "GO:0006886"
}